{
  "term_id": "UNKNOWN:0001",
  "gene_name": "Histone H2A.N",
  "term_label": "Unknown molecular function",
  "gene": "UniProtKB:P0DW85",
  "gene_symbol": "H2BN1"
}